G protein-coupled glutamate receptor signaling pathway [GO:0007216] (biological process) Definition: A G protein-coupled receptor signaling pathway initiated by glutamate binding to its receptor on the surface of a target cell, and ending with the regulation of a downstream cellular process. Relationships: is a type of G protein-coupled receptor signaling pathway [GO:0007186]; is a type of glutamate receptor signaling pathway [GO:0007215]; has part GO:0098988 References: PMID:9131252 Sources: GOC:mah, GOC:signaling Subtypes: GO:0007196, phospholipase C-activating G protein-coupled glutamate receptor signaling pathway [GO:0007206] Also known as: G-protein coupled glutamate receptor signaling pathway, metabotropic glutamate receptor signaling pathway, metabotropic glutamate receptor signalling pathway